protein localization to mitotic spindle pole body [GO:1902440] (biological process) Definition: A process in which a protein is transported to, or maintained in, a location within a mitotic spindle pole body. Subtypes: GO:1990976 References: PMID:22438582 Sources: GOC:TermGenie Relationships: is a type of protein localization to spindle pole body [GO:0071988] Regulation: regulated by regulation of protein localization to mitotic spindle pole body [GO:1902542]; negatively regulated by GO:1902543 Also known as: protein localisation in mitotic spindle pole body, protein localisation to mitotic spindle pole body, protein localization in mitotic spindle pole body, establishment of protein localization to mitotic spindle pole body